{
  "term_label": "sarcomere organization",
  "gene_symbol": "CSRP1",
  "gene_name": "Cysteine and glycine-rich protein 1",
  "gene": "UniProtKB:P21291",
  "term_id": "GO:0045214"
}